{
  "gene": "UniProtKB:Q8N7U6",
  "term_id": "GO:2001256",
  "gene_symbol": "EFHB",
  "gene_name": "EF-hand domain-containing family member B",
  "term_label": "regulation of store-operated calcium entry"
}